positive regulation of phospholipid metabolic process [GO:1903727] (biological process) Relationships: is a type of positive regulation of lipid metabolic process [GO:0045834]; is a type of positive regulation of phosphate metabolic process [GO:0045937]; is a type of regulation of phospholipid metabolic process [GO:1903725]; positively regulates phospholipid metabolic process [GO:0006644] Definition: Any process that activates or increases the frequency, rate or extent of phospholipid metabolic process. Subtypes: GO:0060697, positive regulation of phospholipid biosynthetic process [GO:0071073], positive regulation of cardiolipin metabolic process [GO:1900210] Also known as: positive regulation of phospholipid metabolism, up regulation of phospholipid metabolic process, up regulation of phospholipid metabolism, up-regulation of phospholipid metabolic process, up-regulation of phospholipid metabolism, upregulation of phospholipid metabolic process, upregulation of phospholipid metabolism, activation of phospholipid metabolic process, activation of phospholipid metabolism References: PMID:10657240 Sources: GOC:TermGenie, GO_REF:0000058